{
  "term_label": "response to ionizing radiation",
  "gene_name": "SOSS complex subunit B2",
  "gene_symbol": "NABP1",
  "gene": "UniProtKB:Q96AH0",
  "term_id": "GO:0010212"
}